{
  "term_id": "GO:0005254",
  "gene": "UniProtKB:P78334",
  "gene_name": "Gamma-aminobutyric acid receptor subunit epsilon",
  "gene_symbol": "GABRE",
  "term_label": "chloride channel activity"
}